{
  "gene_symbol": "SGCG",
  "term_label": "heart contraction",
  "term_id": "GO:0060047",
  "gene": "UniProtKB:Q13326",
  "gene_name": "Gamma-sarcoglycan"
}